{
  "gene": "UniProtKB:Q9BYZ6",
  "gene_name": "Rho-related BTB domain-containing protein 2",
  "term_id": "GO:0042995",
  "term_label": "cell projection",
  "gene_symbol": "RHOBTB2"
}